{
  "term_id": "GO:0038023",
  "gene": "UniProtKB:Q86VH4",
  "gene_name": "Leucine-rich repeat transmembrane neuronal protein 4",
  "gene_symbol": "LRRTM4",
  "term_label": "signaling receptor activity"
}